vetispiradiene synthase activity [GO:0034003] (molecular function) Relationships: is a type of sesquiterpene synthase activity [GO:0010334] Also known as: HVS, pemnaspirodiene synthase activity, trans,trans-farnesyl-diphosphate diphosphate-lyase (cyclizing, vetispiradiene-forming) activity, vetispiradiene cyclase activity, vetispiradiene-forming farnesyl pyrophosphate cyclase activity Sources: EC:4.2.3.21, RHEA:10340 Definition: Catalysis of the reaction: 2-trans,6-trans-farnesyl diphosphate = diphosphate + vetispiradiene.